{
  "gene_name": "C-terminal-binding protein 1",
  "gene": "UniProtKB:Q13363",
  "gene_symbol": "CTBP1",
  "term_id": "GO:0140297",
  "term_label": "DNA-binding transcription factor binding"
}